{
  "gene": "UniProtKB:Q4KMQ2",
  "term_label": "calcium activated phosphatidylserine scrambling",
  "gene_name": "Anoctamin-6",
  "term_id": "GO:0061589",
  "gene_symbol": "ANO6"
}